angiotensin-activated signaling pathway involved in heart process [GO:0086098] (biological process) Relationships: is a type of angiotensin-activated signaling pathway [GO:0038166]; is a type of G protein-coupled receptor signaling pathway involved in heart process [GO:0086103] Definition: An angiotensin receptor signaling pathway which contributes to a circulatory system process carried out by the heart. Subtypes: phospholipase C-activating angiotensin-activated signaling pathway involved in heart process [GO:0086099] References: PMID:17376402 Sources: GOC:BHF, GOC:mtg_cardiac_conduct_nov11 Also known as: angiotensin receptor signaling pathway involved in heart process, angiotensin receptor signalling pathway involved in heart process, angiotensin-mediated signaling pathway involved in heart process